{
  "gene_name": "Catenin delta-1",
  "gene": "UniProtKB:O60716",
  "term_id": "GO:0098609",
  "term_label": "cell-cell adhesion",
  "gene_symbol": "CTNND1"
}